{
  "term_id": "GO:0008064",
  "gene_symbol": "NAA80",
  "term_label": "regulation of actin polymerization or depolymerization",
  "gene_name": "N-alpha-acetyltransferase 80",
  "gene": "UniProtKB:Q93015"
}